{
  "gene_symbol": "ZNF799",
  "gene_name": "Zinc finger protein 799",
  "term_id": "GO:0000977",
  "gene": "UniProtKB:Q96GE5",
  "term_label": "RNA polymerase II transcription regulatory region sequence-specific DNA binding"
}